{
  "term_label": "nucleus",
  "gene_symbol": "CTCFL",
  "gene_name": "Transcriptional repressor CTCFL",
  "term_id": "GO:0005634",
  "gene": "UniProtKB:Q8NI51"
}